{
  "term_label": "cytosol",
  "term_id": "GO:0005829",
  "gene_name": "Ubiquitin carboxyl-terminal hydrolase 17-like protein 11",
  "gene_symbol": "USP17L11",
  "gene": "UniProtKB:C9JVI0"
}